fruit replum development [GO:1990058] (biological process) Definition: The process whose specific outcome is the progression of the fruit replum over time, from its formation to the mature structure. The fruit replum is a portion of fruit placenta tissue that divides a fruit into two or more chambers and develops from a replum. References: PMID:23133401 Sources: PO:0025267 Relationships: is a type of post-embryonic development [GO:0009791]; is a type of GO:0048856; is part of GO:0010154